{
  "gene_name": "Low-density lipoprotein receptor-related protein 2",
  "gene": "UniProtKB:P98164",
  "gene_symbol": "LRP2",
  "term_label": "receptor complex",
  "term_id": "GO:0043235"
}